{
  "gene": "UniProtKB:Q9Y4C0",
  "term_label": "neuroligin family protein binding",
  "gene_name": "Neurexin-3",
  "term_id": "GO:0097109",
  "gene_symbol": "NRXN3"
}